tendon sheath development [GO:0002932] (biological process) References: PMID:20696843 Relationships: is_a connective tissue development [GO:0061448]; is part of tendon development [GO:0035989] Definition: The process whose specific outcome is the progression of a tendon sheath over time, from its formation to the mature structure. A tendon sheath is a layer of membrane around a tendon. It permits the tendon to move.